{
  "term_label": "Unknown cellular component",
  "gene": "UniProtKB:Q8WWZ4",
  "gene_name": "ATP-binding cassette sub-family A member 10",
  "gene_symbol": "ABCA10",
  "term_id": "UNKNOWN:0003"
}